{
  "gene": "UniProtKB:O75943",
  "gene_symbol": "RAD17",
  "gene_name": "Cell cycle checkpoint protein RAD17",
  "term_label": "chromosome, telomeric repeat region",
  "term_id": "GO:0140445"
}